{
  "gene": "UniProtKB:O15254",
  "gene_symbol": "ACOX3",
  "term_id": "GO:0005777",
  "term_label": "peroxisome",
  "gene_name": "Peroxisomal acyl-coenzyme A oxidase 3"
}